{
  "term_id": "UNKNOWN:0002",
  "gene_name": "Transmembrane protein 255B",
  "term_label": "Unknown biological process",
  "gene_symbol": "TMEM255B",
  "gene": "UniProtKB:Q8WV15"
}